{
  "gene": "UniProtKB:Q9HD64",
  "gene_symbol": "XAGE1B",
  "term_id": "UNKNOWN:0003",
  "term_label": "Unknown cellular component",
  "gene_name": "X antigen family member 1"
}